{
  "term_id": "GO:0030672",
  "gene": "UniProtKB:Q9UPW8",
  "term_label": "synaptic vesicle membrane",
  "gene_symbol": "UNC13A",
  "gene_name": "Protein unc-13 homolog A"
}